{
  "gene": "UniProtKB:Q9NUL3",
  "gene_name": "Double-stranded RNA-binding protein Staufen homolog 2",
  "term_label": "protein localization to synapse",
  "gene_symbol": "STAU2",
  "term_id": "GO:0035418"
}